{
  "gene_symbol": "SYNM",
  "term_label": "intermediate filament binding",
  "gene_name": "Synemin",
  "gene": "UniProtKB:O15061",
  "term_id": "GO:0019215"
}